histone H2A acetyltransferase activity [GO:0043998] (molecular function) References: PMID:19056256 Relationships: is a type of histone acetyltransferase activity [GO:0004402] Definition: Catalysis of the reaction: acetyl-CoA + histone H2A L-lysine = CoA + histone H2A N6-acetyl-L-lysine. Subtypes: histone H2AK5 acetyltransferase activity [GO:0043999], histone H2AK9 acetyltransferase activity [GO:0044012] Also known as: H2A histone acetylase activity, H2A histone acetyltransferase activity, H2A histone lysine N-acetyltransferase activity